{
  "term_label": "Unknown biological process",
  "gene_symbol": "TMEM145",
  "term_id": "UNKNOWN:0002",
  "gene_name": "Transmembrane protein 145",
  "gene": "UniProtKB:Q8NBT3"
}